glycosyl compound biosynthetic process [GO:1901659] (BP) Relationships: is_a carbohydrate derivative biosynthetic process [GO:1901137] Subtypes: nucleoside biosynthetic process [GO:0009163], glycoside biosynthetic process [GO:0016138], S-glycoside biosynthetic process [GO:0016144], wybutosine biosynthetic process [GO:0031591] Also known as: glycosyl compound anabolism, glycosyl compound biosynthesis, glycosyl compound formation, glycosyl compound synthesis Sources: GOC:TermGenie, GOC:pr Definition: The chemical reactions and pathways resulting in the formation of glycosyl compound.